arsonoacetate catabolic process [GO:0019501] (biological process) Sources: GOC:jl Relationships: is a type of arsonoacetate metabolic process [GO:0018872]; is a type of xenobiotic catabolic process [GO:0042178]; is a type of carboxylic acid catabolic process [GO:0046395] Definition: The chemical reactions and pathways resulting in the breakdown of arsonoacetate, a synthetic, organic compound containing a single arsenic atom. Also known as: arsonoacetate breakdown, arsonoacetate catabolism, arsonoacetate degradation